{
  "gene": "UniProtKB:Q9Y6Q1",
  "gene_name": "Calpain-6",
  "gene_symbol": "CAPN6",
  "term_id": "UNKNOWN:0001",
  "term_label": "Unknown molecular function"
}